{
  "gene_symbol": "IGLC1",
  "gene": "UniProtKB:P0CG04",
  "term_label": "immunoglobulin mediated immune response",
  "gene_name": "Immunoglobulin lambda constant 1",
  "term_id": "GO:0016064"
}